positive regulation of astrocyte activation [GO:0061890] (biological process) Relationships: is a type of positive regulation of astrocyte differentiation [GO:0048711]; is a type of GO:0050867; is a type of regulation of astrocyte activation [GO:0061888]; is a type of GO:0150078; positively regulates astrocyte activation [GO:0048143] References: PMID:20005821 Sources: GOC:aruk, GOC:bc Definition: Any process that increases the frequency, rate or extent of astrocyte activation.